{
  "gene": "UniProtKB:P49588",
  "gene_name": "Alanine--tRNA ligase, cytoplasmic",
  "term_id": "GO:0005829",
  "gene_symbol": "AARS1",
  "term_label": "cytosol"
}